{
  "gene": "UniProtKB:P01737",
  "gene_symbol": "TRAV8-4",
  "term_id": "UNKNOWN:0001",
  "gene_name": "T cell receptor alpha variable 8-4",
  "term_label": "Unknown molecular function"
}